{
  "gene_name": "Ribosomal protein uL30-like",
  "term_id": "GO:0000463",
  "gene": "UniProtKB:Q6DKI1",
  "gene_symbol": "RPL7L1",
  "term_label": "maturation of LSU-rRNA from tricistronic rRNA transcript (SSU-rRNA, 5.8S rRNA, LSU-rRNA)"
}